{
  "gene": "UniProtKB:Q9H9S0",
  "term_label": "regulation of transcription by RNA polymerase II",
  "term_id": "GO:0006357",
  "gene_name": "Homeobox protein NANOG",
  "gene_symbol": "NANOG"
}